{
  "term_label": "chromatin",
  "gene": "UniProtKB:Q8WYB5",
  "gene_name": "Histone acetyltransferase KAT6B",
  "term_id": "GO:0000785",
  "gene_symbol": "KAT6B"
}